{
  "gene_name": "Tribbles homolog 2",
  "gene": "UniProtKB:Q92519",
  "term_id": "GO:0005634",
  "term_label": "nucleus",
  "gene_symbol": "TRIB2"
}